{
  "term_label": "Unknown biological process",
  "gene_name": "Putative protein FAM86C1P",
  "term_id": "UNKNOWN:0002",
  "gene": "UniProtKB:Q9NVL1",
  "gene_symbol": "FAM86C1P"
}